{
  "term_id": "UNKNOWN:0001",
  "gene": "UniProtKB:Q9BZ81",
  "gene_symbol": "MAGEB5",
  "term_label": "Unknown molecular function",
  "gene_name": "Melanoma-associated antigen B5"
}